{
  "gene_name": "N(6)-adenine-specific methyltransferase METTL4",
  "term_id": "GO:0005829",
  "term_label": "cytosol",
  "gene_symbol": "METTL4",
  "gene": "UniProtKB:Q8N3J2"
}